{
  "gene": "UniProtKB:Q8WY50",
  "term_label": "Unknown biological process",
  "gene_symbol": "PLAC4",
  "term_id": "UNKNOWN:0002",
  "gene_name": "Placenta-specific protein 4"
}